{
  "term_id": "GO:0004843",
  "gene_name": "Tumor necrosis factor alpha-induced protein 3",
  "gene_symbol": "TNFAIP3",
  "gene": "UniProtKB:P21580",
  "term_label": "cysteine-type deubiquitinase activity"
}